regulation of steroid hormone biosynthetic process [GO:0090030] (biological process) Definition: Any process that modulates the frequency, rate or extent of the chemical reactions and pathways resulting in the formation of steroid hormones,compounds with a 1, 2, cyclopentanoperhydrophenanthrene nucleus that act as hormones. Sources: GOC:dph, GOC:tb Relationships: is a type of GO:0046885; is_a regulation of steroid biosynthetic process [GO:0050810] Subtypes: regulation of ecdysteroid biosynthetic process [GO:0007554], regulation of brassinosteroid biosynthetic process [GO:0010422], regulation of glucocorticoid biosynthetic process [GO:0031946], GO:0032347, positive regulation of steroid hormone biosynthetic process [GO:0090031], negative regulation of steroid hormone biosynthetic process [GO:0090032]